intermediate mesodermal cell differentiation [GO:0048392] (biological process) Definition: The process in which a relatively unspecialized cell acquires specialized features of an intermediate mesoderm cell. Relationships: is a type of mesodermal cell differentiation [GO:0048333]; is part of GO:0048391 Also known as: intermediate mesoderm cell differentiation Sources: GOC:dgh